{
  "term_id": "GO:0005886",
  "gene_symbol": "ANPEP",
  "term_label": "plasma membrane",
  "gene_name": "Aminopeptidase N",
  "gene": "UniProtKB:P15144"
}